{
  "gene_symbol": "AIP",
  "gene_name": "AH receptor-interacting protein",
  "gene": "UniProtKB:O00170",
  "term_label": "Unknown cellular component",
  "term_id": "UNKNOWN:0003"
}